{
  "gene": "UniProtKB:X6R8R1",
  "gene_name": "Synaptotagmin-15B",
  "term_id": "GO:0016192",
  "gene_symbol": "SYT15B",
  "term_label": "vesicle-mediated transport"
}